{
  "gene": "UniProtKB:Q9C0B6",
  "term_id": "GO:0005737",
  "gene_name": "BMP_retinoic acid-inducible neural-specific protein 2",
  "gene_symbol": "BRINP2",
  "term_label": "cytoplasm"
}